{
  "gene_name": "Guanylate cyclase soluble subunit beta-2",
  "gene_symbol": "GUCY1B2",
  "term_label": "response to oxygen levels",
  "term_id": "GO:0070482",
  "gene": "UniProtKB:O75343"
}